{
  "gene_name": "Calcium-binding and spermatid-specific protein 1",
  "term_label": "mitochondrial inner membrane",
  "gene_symbol": "CABS1",
  "gene": "UniProtKB:Q96KC9",
  "term_id": "GO:0005743"
}